{
  "gene_name": "Cadherin-18",
  "gene_symbol": "CDH18",
  "term_label": "cell-cell junction assembly",
  "term_id": "GO:0007043",
  "gene": "UniProtKB:Q13634"
}